{
  "gene_name": "Aquaporin-7B",
  "gene": "UniProtKB:A0A075B734",
  "term_label": "glycerol channel activity",
  "term_id": "GO:0015254",
  "gene_symbol": "AQP7B"
}